glucose 6-phosphate metabolic process [GO:0051156] (biological process) Relationships: is a type of phosphate-containing compound metabolic process [GO:0006796]; is a type of organophosphate metabolic process [GO:0019637]; is a type of carbohydrate derivative metabolic process [GO:1901135] Sources: GOC:ai Subtypes: pentose-phosphate shunt [GO:0006098], sucrose catabolic process to fructose-6-phosphate and glucose-6-phosphate [GO:0036008] Definition: The chemical reactions and pathways involving glucose 6-phosphate, a monophosphorylated derivative of glucose with the phosphate group attached to C-6. Also known as: glucose 6-phosphate metabolism, glucose 6-phosphate utilization